{
  "term_id": "UNKNOWN:0002",
  "gene": "UniProtKB:P55040",
  "term_label": "Unknown biological process",
  "gene_name": "GTP-binding protein GEM",
  "gene_symbol": "GEM"
}